{
  "gene_symbol": "SHANK3",
  "term_id": "GO:0030160",
  "gene": "UniProtKB:Q9BYB0",
  "term_label": "synaptic receptor adaptor activity",
  "gene_name": "SH3 and multiple ankyrin repeat domains protein 3"
}